negative regulation of cumulus cell differentiation [GO:0045593] (biological process) Relationships: is a type of GO:0030857; is_a regulation of cumulus cell differentiation [GO:0045592]; is a type of negative regulation of reproductive process [GO:2000242]; negatively regulates cumulus cell differentiation [GO:0001549] Definition: Any process that stops, prevents, or reduces the frequency, rate or extent of ovarian cumulus cell differentiation. Sources: GOC:go_curators Also known as: down regulation of cumulus cell differentiation, down-regulation of cumulus cell differentiation, downregulation of cumulus cell differentiation, negative regulation of ovarian cumulus cell differentiation, inhibition of cumulus cell differentiation